{
  "term_label": "sprouting angiogenesis",
  "gene_symbol": "VEGFC",
  "gene_name": "Vascular endothelial growth factor C",
  "term_id": "GO:0002040",
  "gene": "UniProtKB:P49767"
}